{
  "gene_symbol": "RTN4RL2",
  "gene": "UniProtKB:Q86UN3",
  "gene_name": "Reticulon-4 receptor-like 2",
  "term_id": "GO:0009897",
  "term_label": "external side of plasma membrane"
}